{
  "gene_name": "Ezrin",
  "term_id": "GO:0045177",
  "gene_symbol": "EZR",
  "term_label": "apical part of cell",
  "gene": "UniProtKB:P15311"
}